{
  "term_id": "GO:2000049",
  "term_label": "positive regulation of cell-cell adhesion mediated by cadherin",
  "gene": "UniProtKB:Q8IWF6",
  "gene_symbol": "DENND6A",
  "gene_name": "Protein DENND6A"
}